glucose import in response to insulin stimulus [GO:0044381] (biological process) Definition: The directed movement of the hexose monosaccharide glucose into a cell as a result of an insulin stimulus. References: PMID:19079291 Sources: GOC:BHF Also known as: cellular glucose import in response to insulin stimulus Relationships: is a type of GO:0046323; is part of cellular response to insulin stimulus [GO:0032869]